neurotransmitter receptor activity [GO:0030594] (molecular function) Subtypes: benzodiazepine receptor activity [GO:0008503], transmitter-gated channel activity [GO:0022835], postsynaptic neurotransmitter receptor activity [GO:0098960], G protein-coupled neurotransmitter receptor activity [GO:0099528], GO:0099582 Regulation: regulated by regulation of neurotransmitter receptor activity [GO:0099601]; regulated by neurotransmitter receptor regulator activity [GO:0099602] Relationships: is a type of signaling receptor activity [GO:0038023] Note: A strict definition of neurotransmitter receptor activity would limit its use to receptor activity at the postsynaptic membrane as part of synaptic transmission, but we recognize that usage is often much broader than this. For the strict use case, please see 'postsynaptic neurotransmitter receptor activity' Definition: Combining with a neurotransmitter and transmitting the signal to initiate a change in cell activity. Sources: GOC:jl, GOC:signaling